alpha DNA polymerase:primase complex [GO:0005658] (cellular component) Definition: A complex of four polypeptides, comprising large and small DNA polymerase alpha subunits and two primase subunits, which are capable of catalyzing the synthesis of an RNA primer on the lagging strand of replicating DNA and the subsequent synthesis of a small stretch of DNA. The smaller of the two primase subunits alone can catalyze oligoribonucleotide synthesis. References: PMID:11395402, PMID:26975377 Sources: GOC:mah Relationships: is a type of DNA polymerase complex [GO:0042575]; is a type of nuclear DNA-directed RNA polymerase complex [GO:0055029]; is part of nuclear replisome [GO:0043601] Also known as: primosome, DNA polymerase alpha:primase complex, heterotetrameric polymerase alpha holoenzyme, pol-prim